{
  "term_label": "chromosome condensation",
  "gene_symbol": "H1-5",
  "term_id": "GO:0030261",
  "gene_name": "Histone H1.5",
  "gene": "UniProtKB:P16401"
}